{
  "term_id": "GO:0016593",
  "term_label": "Cdc73/Paf1 complex",
  "gene_name": "Parafibromin",
  "gene": "UniProtKB:Q6P1J9",
  "gene_symbol": "CDC73"
}